{
  "gene_symbol": "CXADR",
  "gene_name": "Coxsackievirus and adenovirus receptor",
  "term_id": "GO:0005923",
  "term_label": "bicellular tight junction",
  "gene": "UniProtKB:P78310"
}